{
  "gene_name": "Trace amine-associated receptor 9",
  "term_id": "GO:0005886",
  "term_label": "plasma membrane",
  "gene_symbol": "TAAR9",
  "gene": "UniProtKB:Q96RI9"
}